{
  "gene": "UniProtKB:P48029",
  "gene_symbol": "SLC6A8",
  "gene_name": "Sodium- and chloride-dependent creatine transporter 1",
  "term_id": "GO:0006865",
  "term_label": "amino acid transport"
}